forebrain neuron differentiation [GO:0021879] (biological process) Regulation: regulated by regulation of forebrain neuron differentiation [GO:2000977]; negatively regulated by GO:2000978; RO_0002213 by GO:2000979 Relationships: is a type of central nervous system neuron differentiation [GO:0021953]; is part of forebrain generation of neurons [GO:0021872] References: PMID:16226447 Sources: GOC:cls, GOC:dgh, GOC:dph, GOC:jid, GO_REF:0000021 Subtypes: GO:0021773, GO:0021862, olfactory bulb interneuron differentiation [GO:0021889], cerebral cortex neuron differentiation [GO:0021895], thyroid-stimulating hormone-secreting cell differentiation [GO:0060129] Definition: The process in which a relatively unspecialized cell acquires specialized features of a neuron that will reside in the forebrain.